{
  "term_label": "RNA polymerase II cis-regulatory region sequence-specific DNA binding",
  "gene_name": "Homeobox protein Hox-A11",
  "gene_symbol": "HOXA11",
  "gene": "UniProtKB:P31270",
  "term_id": "GO:0000978"
}